{
  "term_id": "GO:0005634",
  "term_label": "nucleus",
  "gene_symbol": "ZFPM2",
  "gene": "UniProtKB:Q8WW38",
  "gene_name": "Zinc finger protein ZFPM2"
}